{
  "gene": "UniProtKB:Q8WUU4",
  "gene_symbol": "ZNF296",
  "term_id": "GO:0003700",
  "gene_name": "Zinc finger protein 296",
  "term_label": "DNA-binding transcription factor activity"
}